{
  "term_label": "response to nutrient levels",
  "term_id": "GO:0031667",
  "gene": "UniProtKB:P0DML2",
  "gene_name": "Chorionic somatomammotropin hormone 1",
  "gene_symbol": "CSH1"
}